{
  "gene": "UniProtKB:Q9Y2W6",
  "term_id": "UNKNOWN:0001",
  "gene_name": "Tudor and KH domain-containing protein",
  "term_label": "Unknown molecular function",
  "gene_symbol": "TDRKH"
}